{
  "term_label": "centrosome",
  "gene_symbol": "CNTLN",
  "gene_name": "Centlein",
  "gene": "UniProtKB:Q9NXG0",
  "term_id": "GO:0005813"
}